{
  "gene_name": "Calpain-15",
  "gene_symbol": "CAPN15",
  "gene": "UniProtKB:O75808",
  "term_id": "GO:0005737",
  "term_label": "cytoplasm"
}